negative regulation of smooth endoplasmic reticulum calcium ion concentration [GO:0051565] (biological process) Definition: Any process that decreases the concentration of calcium ions in the smooth endoplasmic reticulum. Sources: GOC:ai Also known as: reduction of calcium ion concentration in smooth ER, reduction of calcium ion concentration in smooth endoplasmic reticulum, reduction of smooth ER calcium ion concentration, reduction of smooth endoplasmic reticulum calcium ion concentration, smooth ER calcium ion concentration reduction, smooth endoplasmic reticulum calcium ion concentration reduction Relationships: is a type of GO:0032471; is a type of GO:0051563